{
  "term_label": "Unknown biological process",
  "gene_symbol": "SSX6P",
  "term_id": "UNKNOWN:0002",
  "gene": "UniProtKB:Q7RTT6",
  "gene_name": "Putative protein SSX6"
}